{
  "gene_symbol": "LYVE1",
  "gene_name": "Lymphatic vessel endothelial hyaluronic acid receptor 1",
  "term_id": "GO:0005540",
  "term_label": "hyaluronic acid binding",
  "gene": "UniProtKB:Q9Y5Y7"
}